RNA-binding transcription regulator activity [GO:0001070] (molecular function) Relationships: is_a transcription regulator activity [GO:0140110]; is part of positive regulation of DNA-templated transcription [GO:0045893]; has part transcription regulatory region RNA binding [GO:0001068] Definition: A transcription regulator activity that modulates the transcription of specific gene sets via selective and non-covalent binding to a specific RNA sequence. This function is known to occur in phages and viruses, for example the lambda N and the HIV tat proteins are necessary to allow RNA polymerase to read through terminator sequences. References: PMID:1756726 Sources: GOC:txnOH-2018 Also known as: RNA binding transcription regulator activity, RNA binding transcription factor activity